mitogen-activated protein kinase binding [GO:0051019] (molecular function) Also known as: MAP kinase binding, MAPK binding, MAP-kinase anchoring activity Relationships: is a type of protein kinase binding [GO:0019901] Definition: Binding to a mitogen-activated protein kinase. Subtypes: mitogen-activated protein kinase p38 binding [GO:0048273] Sources: GOC:ai